regulation of (1->3)-beta-D-glucan biosynthetic process [GO:0032953] (biological process) Definition: Any process that modulates the frequency, rate or extent of the chemical reactions and pathways resulting in the formation of (1->3)-beta-D-glucans. Sources: GOC:mah Also known as: regulation of 1,3-beta-glucan biosynthetic process, regulation of 1,3-beta-glucan anabolism, regulation of 1,3-beta-glucan biosynthesis, regulation of 1,3-beta-glucan formation, regulation of 1,3-beta-glucan synthesis Relationships: is a type of regulation of beta-glucan biosynthetic process [GO:0032951]; RO_0002211 (1->3)-beta-D-glucan biosynthetic process [GO:0006075] Subtypes: positive regulation of (1->3)-beta-D-glucan biosynthetic process [GO:0060635], GO:0060636, GO:0090334